{
  "term_label": "Unknown molecular function",
  "gene": "UniProtKB:Q9NQ60",
  "gene_symbol": "EQTN",
  "gene_name": "Equatorin",
  "term_id": "UNKNOWN:0001"
}